{
  "gene_symbol": "EXOSC9",
  "gene_name": "Exosome complex component RRP45",
  "gene": "UniProtKB:Q06265",
  "term_id": "GO:0034475",
  "term_label": "U4 snRNA 3'-end processing"
}